{
  "gene_symbol": "A0A8I5KYW3",
  "term_id": "UNKNOWN:0003",
  "gene_name": "Uncharacterized protein",
  "term_label": "Unknown cellular component",
  "gene": "UniProtKB:A0A8I5KYW3"
}